{
  "term_id": "GO:0005035",
  "gene": "UniProtKB:P08138",
  "term_label": "death receptor activity",
  "gene_symbol": "NGFR",
  "gene_name": "Tumor necrosis factor receptor superfamily member 16"
}